{
  "gene_name": "Putative protein FAM90A8",
  "gene": "UniProtKB:A6NJQ4",
  "term_id": "UNKNOWN:0001",
  "gene_symbol": "FAM90A8",
  "term_label": "Unknown molecular function"
}